{
  "gene_symbol": "MBL2",
  "gene_name": "Mannose-binding protein C",
  "gene": "UniProtKB:P11226",
  "term_id": "UNKNOWN:0001",
  "term_label": "Unknown molecular function"
}